jasmonic acid hydrolase [GO:0120091] (MF) Also known as: 2-oxoglutarate dioxygenase Relationships: is a type of hydrolase activity, acting on carbon-nitrogen (but not peptide) bonds [GO:0016810] References: PMID:28559313, PMID:28760569 Definition: Catalyzes the hydroxylation of jasmonic acid to 12OH-jasmonic acid.